{
  "gene_name": "Spermatogenesis-associated protein 13",
  "term_label": "lamellipodium assembly",
  "term_id": "GO:0030032",
  "gene": "UniProtKB:Q96N96",
  "gene_symbol": "SPATA13"
}